{
  "term_label": "Unknown molecular function",
  "gene_symbol": "TRABD",
  "gene_name": "TraB domain-containing protein",
  "gene": "UniProtKB:Q9H4I3",
  "term_id": "UNKNOWN:0001"
}